{
  "gene_symbol": "PPDPF",
  "gene_name": "Pancreatic progenitor cell differentiation and proliferation factor",
  "term_id": "UNKNOWN:0003",
  "gene": "UniProtKB:Q9H3Y8",
  "term_label": "Unknown cellular component"
}